{
  "gene_name": "Eukaryotic translation initiation factor 3 subunit H",
  "gene_symbol": "EIF3H",
  "term_id": "GO:0003743",
  "term_label": "translation initiation factor activity",
  "gene": "UniProtKB:O15372"
}